{
  "gene_name": "Taste receptor type 2 member 8",
  "term_id": "GO:0016020",
  "gene": "UniProtKB:Q9NYW2",
  "gene_symbol": "TAS2R8",
  "term_label": "membrane"
}